protein guanylylation [GO:0018260] (biological process) Definition: The addition of phospho-guanosine to a protein amino acid. Relationships: is a type of protein nucleotidylation [GO:0018175] Sources: GOC:ai Also known as: protein amino acid guanylylation